DCT cell fate commitment [GO:0072146] (biological process) Also known as: distal convoluted tubule cell fate commitment Subtypes: metanephric DCT cell fate commitment [GO:0072242] Relationships: is a type of cell fate commitment [GO:0045165]; is part of DCT cell differentiation [GO:0072069] Definition: The process in which the developmental fate of a cell becomes restricted such that it will develop into a distal convoluted tubule cell. Sources: GOC:mtg_kidney_jan10